4-hydroxyphenylacetate metabolic process [GO:1901022] (biological process) Also known as: 4-hydroxyphenylacetate metabolism Definition: The chemical reactions and pathways involving 4-hydroxyphenylacetate. Subtypes: 4-hydroxyphenylacetate catabolic process [GO:1901023], 4-hydroxyphenylacetate biosynthetic process [GO:1901024] Relationships: is a type of phenol-containing compound metabolic process [GO:0018958]; is a type of monocarboxylic acid metabolic process [GO:0032787] Sources: GOC:TermGenie, GOC:yaf